{
  "gene_name": "Endosialin",
  "term_label": "cell migration",
  "gene_symbol": "CD248",
  "term_id": "GO:0016477",
  "gene": "UniProtKB:Q9HCU0"
}